{
  "gene": "UniProtKB:P21754",
  "term_id": "GO:0035804",
  "gene_name": "Zona pellucida sperm-binding protein 3",
  "gene_symbol": "ZP3",
  "term_label": "structural constituent of egg coat"
}